1,8-cineole synthase activity [GO:0102313] (molecular function) Relationships: is a type of carbon-oxygen lyase activity, acting on phosphates [GO:0016838] Definition: Catalysis of the reaction: geranyl diphosphate(3-) + H2O = 1,8-cineole + diphosphoric acid. Sources: GOC:pz, RHEA:32543